cellular response to anoxia [GO:0071454] (biological process) Relationships: is a type of cellular response to stress [GO:0033554]; is_a GO:0034059; is_a cellular response to decreased oxygen levels [GO:0036294] Definition: Any process that results in a change in state or activity of a cell (in terms of movement, secretion, enzyme production, gene expression, etc.) as a result of a stimulus indicating a decline in oxygen levels to trace amounts, <0.1%. Also known as: cellular response to anaerobic conditions, cellular response to anoxic stress Note: Note that this term should not be confused with 'cellular response to hypoxia ; GO:0071456'. Sources: GOC:mah